nucleus-vacuole junction assembly [GO:0071562] (biological process) Relationships: is_a cellular component assembly [GO:0022607]; is_a organelle localization by membrane tethering [GO:0140056] References: PMID:16709156, PMID:28533415 Sources: GOC:jp Definition: The aggregation, arrangement and bonding together of a set of components to form a nucleus-vacuole junction (NVJ), membrane contact sites formed between the vacuole membrane and the outer nuclear membrane. In S. cerevisiae these contacts are mediated through direct physical interaction between Vac8p and Nvj1p. The NVJ plays roles in piecemeal microautophagy of the nucleus and in the cytoplasm-to-vacuole targeting pathway. Also known as: NV junction assembly, NV junction formation, NVJ assembly, NVJ formation, nucleus-vacuole junction formation